{
  "term_label": "DNA-binding transcription factor activity, RNA polymerase II-specific",
  "term_id": "GO:0000981",
  "gene_name": "Zinc finger protein 394",
  "gene": "UniProtKB:Q53GI3",
  "gene_symbol": "ZNF394"
}